negative regulation of epithelial to mesenchymal transition [GO:0010719] (biological process) Sources: GOC:BHF, GOC:dph, GOC:tb Relationships: is a type of GO:0010717; is a type of negative regulation of cell differentiation [GO:0045596]; is a type of GO:0051241; negatively regulates epithelial to mesenchymal transition [GO:0001837] Definition: Any process that decreases the rate, frequency, or extent of epithelial to mesenchymal transition. Epithelial to mesenchymal transition where an epithelial cell loses apical/basolateral polarity, severs intercellular adhesive junctions, degrades basement membrane components and becomes a migratory mesenchymal cell. Subtypes: GO:0062044, GO:0090301